{
  "term_label": "DNA replication proofreading",
  "term_id": "GO:0045004",
  "gene": "UniProtKB:Q07864",
  "gene_symbol": "POLE",
  "gene_name": "DNA polymerase epsilon catalytic subunit A"
}